regulation of post-transcriptional gene silencing [GO:0060147] (BP) Definition: Any process that modulates the frequency, rate or extent of the inactivation of gene expression by a posttranscriptional mechanism. Sources: GOC:dph Also known as: regulation of posttranscriptional gene silencing Relationships: is a type of regulation of gene expression [GO:0010468]; regulates GO:0016441 Subtypes: positive regulation of post-transcriptional gene silencing [GO:0060148], negative regulation of post-transcriptional gene silencing [GO:0060149], regulation of post-transcriptional gene silencing by regulatory ncRNA [GO:1900368]